{
  "gene_symbol": "DGKZ",
  "term_id": "GO:0004143",
  "gene_name": "Diacylglycerol kinase zeta",
  "term_label": "ATP-dependent diacylglycerol kinase activity",
  "gene": "UniProtKB:Q13574"
}